{
  "gene": "UniProtKB:Q9NXR8",
  "gene_symbol": "ING3",
  "term_id": "UNKNOWN:0001",
  "gene_name": "Inhibitor of growth protein 3",
  "term_label": "Unknown molecular function"
}